{
  "gene_symbol": "PPCS",
  "term_label": "nucleus",
  "gene_name": "Phosphopantothenate--cysteine ligase",
  "term_id": "GO:0005634",
  "gene": "UniProtKB:Q9HAB8"
}